{
  "term_label": "guanyl-nucleotide exchange factor activity",
  "gene_symbol": "RAPGEF1",
  "gene_name": "Rap guanine nucleotide exchange factor 1",
  "term_id": "GO:0005085",
  "gene": "UniProtKB:Q13905"
}